{
  "term_id": "GO:0031647",
  "gene": "UniProtKB:C9J2P7",
  "gene_symbol": "USP17L15",
  "term_label": "regulation of protein stability",
  "gene_name": "Ubiquitin carboxyl-terminal hydrolase 17-like protein 15"
}